{
  "gene_symbol": "XKR6",
  "gene_name": "XK-related protein 6",
  "gene": "UniProtKB:Q5GH73",
  "term_label": "phosphatidylserine exposure on apoptotic cell surface",
  "term_id": "GO:0070782"
}